polkadots [GO:0002096] (cellular component) Definition: A punctate, filamentous structure composed of Bcl10 that appears in the cytoplasm of T-cells shortly after T-cell receptor stimulation. Polkadots stands for Punctate Oligomeric Killing and Activating DOmains Transducing Signals. References: PMID:14724296, PMID:16495340 Note: Note that polkadots also contains some amount of MALT1. Interaction with MALT1 is required for formation of the polkadots. Relationships: is a type of protein-containing complex [GO:0032991]; is part of GO:0005737